positive regulation of collagen metabolic process [GO:0010714] (biological process) Relationships: is a type of positive regulation of metabolic process [GO:0009893]; is a type of regulation of collagen metabolic process [GO:0010712]; positively regulates collagen metabolic process [GO:0032963] Subtypes: positive regulation of collagen biosynthetic process [GO:0032967], positive regulation of collagen catabolic process [GO:0120158] Definition: Any process that increases the frequency, rate or extent of the chemical reactions and pathways resulting in the metabolism of collagen, any of a group of fibrous proteins of very high tensile strength that form the main component of connective tissue in animals. Also known as: positive regulation of collagen metabolism Sources: GOC:dph, GOC:tb